{
  "gene": "UniProtKB:Q13609",
  "gene_name": "Deoxyribonuclease gamma",
  "term_label": "apoptotic DNA fragmentation",
  "term_id": "GO:0006309",
  "gene_symbol": "DNASE1L3"
}